{
  "gene": "UniProtKB:P03901",
  "term_label": "Unknown molecular function",
  "term_id": "UNKNOWN:0001",
  "gene_name": "NADH-ubiquinone oxidoreductase chain 4L",
  "gene_symbol": "MT-ND4L"
}